{
  "term_label": "actin cytoskeleton",
  "gene": "UniProtKB:P0CG39",
  "gene_name": "POTE ankyrin domain family member J",
  "gene_symbol": "POTEJ",
  "term_id": "GO:0015629"
}